{
  "term_id": "GO:0043548",
  "gene_symbol": "IRS4",
  "term_label": "phosphatidylinositol 3-kinase binding",
  "gene_name": "Insulin receptor substrate 4",
  "gene": "UniProtKB:O14654"
}